{
  "gene_name": "NADH dehydrogenase [ubiquinone] 1 subunit C1, mitochondrial",
  "gene_symbol": "NDUFC1",
  "gene": "UniProtKB:O43677",
  "term_id": "GO:0045271",
  "term_label": "respiratory chain complex I"
}